inhibin B complex [GO:0043513] (cellular component) Relationships: is a type of GO:0043511 Note: Note that the actions of the inhibin complex are the opposite of those of the activin complex, which is a dimer of an inhibin beta-A and/or inhibin beta-B subunit. See also the cellular component term 'activin complex ; GO:0048180'. Sources: GOC:jl Definition: Heterodimeric hormone composed of an inhibin alpha subunit complexed with an inhibin beta-B subunit.